{
  "gene": "UniProtKB:Q9BR39",
  "gene_symbol": "JPH2",
  "term_label": "junctional membrane complex",
  "gene_name": "Junctophilin-2",
  "term_id": "GO:0030314"
}